{
  "gene": "UniProtKB:Q0P6D2",
  "gene_name": "Divergent protein kinase domain 1C",
  "gene_symbol": "DIPK1C",
  "term_label": "Unknown molecular function",
  "term_id": "UNKNOWN:0001"
}